{
  "term_id": "GO:0043014",
  "term_label": "alpha-tubulin binding",
  "gene_name": "Protein FAM110C",
  "gene_symbol": "FAM110C",
  "gene": "UniProtKB:Q1W6H9"
}